{
  "term_id": "GO:0005886",
  "gene": "UniProtKB:Q9BXC1",
  "gene_name": "Probable G-protein coupled receptor 174",
  "gene_symbol": "GPR174",
  "term_label": "plasma membrane"
}